regulation of retinal rod cell fate commitment [GO:0060224] (biological process) Subtypes: GO:0060225 Relationships: is a type of regulation of cell fate commitment [GO:0010453]; is a type of GO:0046532; regulates retinal rod cell fate commitment [GO:0060223] Sources: GOC:dph Definition: Any process that modulates the process in which the developmental fate of a cell becomes restricted such that it will develop into a retinal rod cell. A retinal rod cell is one of the two photoreceptor subtypes in a camera-type eye.